negative regulation of animal organ morphogenesis [GO:0110111] (biological process) Definition: Any process that stops, prevents, or reduces the frequency, rate or extent of animal organ morphogenesis. Relationships: is a type of negative regulation of developmental process [GO:0051093]; is a type of negative regulation of multicellular organismal process [GO:0051241]; is a type of regulation of animal organ morphogenesis [GO:2000027]; RO_0002212 animal organ morphogenesis [GO:0009887] Sources: GOC:kmv Subtypes: negative regulation of odontogenesis [GO:0042483], GO:0110042, GO:1904119